{
  "gene": "UniProtKB:Q6P4D5",
  "term_id": "GO:0005737",
  "gene_symbol": "PABIR3",
  "term_label": "cytoplasm",
  "gene_name": "PABIR family member 1"
}